{
  "term_id": "GO:0005737",
  "gene_symbol": "DUSP16",
  "term_label": "cytoplasm",
  "gene_name": "Dual specificity protein phosphatase 16",
  "gene": "UniProtKB:Q9BY84"
}